flavin adenine dinucleotide metabolic process [GO:0072387] (biological process) Relationships: is a type of nucleotide metabolic process [GO:0009117]; is a type of flavin-containing compound metabolic process [GO:0042726] Also known as: FAD or FADH2 metabolic process, flavin adenine dinucleotide metabolism, flavin-adenine dinucleotide metabolic process Definition: The chemical reactions and pathways involving flavin adenine dinucleotide, which acts as a coenzyme or prosthetic group of various flavoprotein oxidoreductase enzymes. Sources: GOC:mah Subtypes: FADH2 metabolic process [GO:0006746], FAD metabolic process [GO:0046443], flavin adenine dinucleotide biosynthetic process [GO:0072388], GO:0072389